gephyrin clustering involved in postsynaptic density assembly [GO:0097116] (biological process) Definition: The clustering process in which gephyrin molecules are localized to distinct domains in the postsynaptic density as part of postsynaptic density assembly. Gephyrin is a component of the postsynaptic protein network of inhibitory synapses. Also known as: Geph clustering Relationships: is a type of protein localization to synapse [GO:0035418]; is part of postsynaptic density assembly [GO:0097107] References: PMID:15620359, PMID:24552784, PMID:25772192 Sources: GOC:BHF, GOC:sjp